{
  "gene_name": "Acetyl-coenzyme A transporter 1",
  "gene": "UniProtKB:O00400",
  "term_label": "acetyl-CoA transmembrane transport",
  "gene_symbol": "SLC33A1",
  "term_id": "GO:0035348"
}